{
  "gene_symbol": "TMEM139",
  "term_id": "UNKNOWN:0003",
  "term_label": "Unknown cellular component",
  "gene": "UniProtKB:Q8IV31",
  "gene_name": "Transmembrane protein 139"
}